phosphinothricin N-acetyltransferase activity [GO:0102971] (molecular function) Relationships: is a type of acyltransferase activity, transferring groups other than amino-acyl groups [GO:0016747] Sources: EC:2.3.1.183, GOC:pz Definition: Catalysis of the reaction: acetyl-CoA + phosphinothricin = H+ + coenzyme A(4-) + N-acetylphosphinatothricinate.